regulation of placenta blood vessel development [GO:0110079] (biological process) References: PMID:27748453 Sources: GOC:BHF, GOC:BHF_miRNA, GOC:rph Relationships: is a type of regulation of vasculature development [GO:1901342]; regulates placenta blood vessel development [GO:0060674] Subtypes: positive regulation of placenta blood vessel development [GO:0110080], negative regulation of placenta blood vessel development [GO:0110081] Definition: Any process that modulates the frequency, rate or extent of placenta blood vessel development.